{
  "gene_symbol": "RDX",
  "gene": "UniProtKB:P35241",
  "term_label": "microvillus",
  "gene_name": "Radixin",
  "term_id": "GO:0005902"
}